negative regulation of amacrine cell differentiation [GO:1902870] (biological process) Definition: Any process that stops, prevents or reduces the frequency, rate or extent of amacrine cell differentiation. Also known as: down regulation of amacrine cell differentiation, down regulation of amacrine neuron differentiation, down-regulation of amacrine cell differentiation, down-regulation of amacrine neuron differentiation, downregulation of amacrine cell differentiation, downregulation of amacrine neuron differentiation, negative regulation of amacrine neuron differentiation, inhibition of amacrine cell differentiation, inhibition of amacrine neuron differentiation Relationships: is_a negative regulation of neuron differentiation [GO:0045665]; is a type of regulation of amacrine cell differentiation [GO:1902869]; negatively regulates amacrine cell differentiation [GO:0035881] References: PMID:16872597 Sources: GOC:TermGenie, GOC:mr, GO_REF:0000058